middle ear morphogenesis [GO:0042474] (biological process) Relationships: is a type of embryonic morphogenesis [GO:0048598]; is part of ear morphogenesis [GO:0042471] Definition: The process in which the anatomical structures of the middle ear are generated and organized. The middle ear is the air-filled cavity within the skull of vertebrates that lies between the outer ear and the inner ear. It is linked to the pharynx (and therefore to outside air) via the Eustachian tube and in mammals contains the three ear ossicles, which transmit auditory vibrations from the outer ear (via the tympanum) to the inner ear (via the oval window). Sources: GOC:jl, ISBN:0192801023